{
  "gene_symbol": "IGKV2-40",
  "gene": "UniProtKB:A0A087WW87",
  "term_id": "GO:0006955",
  "term_label": "immune response",
  "gene_name": "Immunoglobulin kappa variable 2-40"
}